IRES-dependent translational initiation of circular RNA [GO:0110019] (biological process) References: PMID:28281539, PMID:28344080, PMID:28344082 Sources: GOC:sp Relationships: is a type of cap-independent translational initiation of circular RNA [GO:0110018]; has part IRES-mediated translation initiation factor activity [GO:0160297] Also known as: IRES-dependent translational initiation of circRNA Definition: The process where translation initiation recruits the 40S ribosomal subunits via an internal ribosome entry segment (IRES) before an AUG codon is encountered in an appropriate sequence context to initiate circular mRNA translation.